{
  "gene_symbol": "KRTAP9-9",
  "term_label": "Unknown molecular function",
  "gene_name": "Keratin-associated protein 9-9",
  "term_id": "UNKNOWN:0001",
  "gene": "UniProtKB:Q9BYP9"
}